{
  "gene_symbol": "RUNDC1",
  "gene_name": "RUN domain-containing protein 1",
  "gene": "UniProtKB:Q96C34",
  "term_label": "Unknown biological process",
  "term_id": "UNKNOWN:0002"
}